{
  "term_id": "GO:0016020",
  "gene_symbol": "DST",
  "term_label": "membrane",
  "gene": "UniProtKB:Q03001",
  "gene_name": "Dystonin"
}